insulin receptor binding [GO:0005158] (molecular function) Also known as: insulin receptor ligand Relationships: is_a GO:0005102 Sources: GOC:ai Definition: Binding to an insulin receptor.